{
  "term_id": "UNKNOWN:0003",
  "gene_symbol": "NLRC4",
  "gene": "UniProtKB:Q9NPP4",
  "term_label": "Unknown cellular component",
  "gene_name": "NLR family CARD domain-containing protein 4"
}